{
  "gene_name": "Membrane-associated guanylate kinase, WW and PDZ domain-containing protein 1",
  "term_id": "GO:0005737",
  "gene": "UniProtKB:Q96QZ7",
  "term_label": "cytoplasm",
  "gene_symbol": "MAGI1"
}